{
  "term_label": "Golgi membrane",
  "term_id": "GO:0000139",
  "gene": "UniProtKB:Q9H2G9",
  "gene_symbol": "BLZF1",
  "gene_name": "Golgin-45"
}